B cell inhibitory signaling pathway [GO:0002773] (biological process) Relationships: is a type of immune response-inhibiting cell surface receptor signaling pathway [GO:0002767] Also known as: B cell inhibitory signalling pathway, B lymphocyte inhibitory signaling pathwayBT-lymphocyte inhibitory signaling pathway, B-cell inhibitory signaling pathway Definition: The series of molecular signals initiated by an extracellular ligand binding to a receptor on the surface of a B cell capable of inhibiting an immune effector process contributing to an immune response. References: PMID:16413920 Sources: GOC:add